{
  "gene_symbol": "RDH13",
  "gene_name": "Retinol dehydrogenase 13",
  "term_label": "eye photoreceptor cell development",
  "gene": "UniProtKB:Q8NBN7",
  "term_id": "GO:0042462"
}